{
  "gene_symbol": "WDR82",
  "gene_name": "WD repeat-containing protein 82",
  "gene": "UniProtKB:Q6UXN9",
  "term_label": "Set1C/COMPASS complex",
  "term_id": "GO:0048188"
}